{
  "gene_symbol": "FAM98C",
  "term_label": "Unknown molecular function",
  "gene": "UniProtKB:Q17RN3",
  "term_id": "UNKNOWN:0001",
  "gene_name": "Protein FAM98C"
}